{
  "gene_name": "Oligophrenin-1",
  "gene": "UniProtKB:O60890",
  "gene_symbol": "OPHN1",
  "term_label": "negative regulation of proteasomal protein catabolic process",
  "term_id": "GO:1901799"
}